cellular response to growth factor stimulus [GO:0071363] (biological process) Regulation: regulated by GO:0090287; negatively regulated by negative regulation of cellular response to growth factor stimulus [GO:0090288] Relationships: is a type of response to growth factor [GO:0070848]; is_a cellular response to endogenous stimulus [GO:0071495] Definition: Any process that results in a change in state or activity of a cell (in terms of movement, secretion, enzyme production, gene expression, etc.) as a result of a growth factor stimulus. Subtypes: cellular response to hepatocyte growth factor stimulus [GO:0035729], cellular response to vascular endothelial growth factor stimulus [GO:0035924], cellular response to platelet-derived growth factor stimulus [GO:0036120], GO:0044344, GO:0071364, cellular response to transforming growth factor beta stimulus [GO:0071560], GO:0071773, cellular response to nerve growth factor stimulus [GO:1990090], GO:1990792 Sources: GOC:mah